positive regulation of tetrapyrrole biosynthetic process from glutamate [GO:1901412] (biological process) Definition: Any process that activates or increases the frequency, rate or extent of tetrapyrrole biosynthetic process from glutamate. Sources: GOC:TermGenie, GOC:mengo_curators Also known as: activation of tetrapyrrole anabolism from glutamate, activation of tetrapyrrole biosynthesis from glutamate, activation of tetrapyrrole formation from glutamate, activation of tetrapyrrole synthesis from glutamate, positive regulation of tetrapyrrole anabolism from glutamate, positive regulation of tetrapyrrole biosynthesis from glutamate, positive regulation of tetrapyrrole formation from glutamate, positive regulation of tetrapyrrole synthesis from glutamate, up regulation of tetrapyrrole anabolism from glutamate, up regulation of tetrapyrrole biosynthesis from glutamate, up regulation of tetrapyrrole biosynthetic process from glutamate, up regulation of tetrapyrrole formation from glutamate, up regulation of tetrapyrrole synthesis from glutamate, up-regulation of tetrapyrrole anabolism from glutamate, up-regulation of tetrapyrrole biosynthesis from glutamate, up-regulation of tetrapyrrole biosynthetic process from glutamate, up-regulation of tetrapyrrole formation from glutamate, up-regulation of tetrapyrrole synthesis from glutamate, upregulation of tetrapyrrole anabolism from glutamate, upregulation of tetrapyrrole biosynthesis from glutamate, upregulation of tetrapyrrole biosynthetic process from glutamate, upregulation of tetrapyrrole formation from glutamate, upregulation of tetrapyrrole synthesis from glutamate, activation of tetrapyrrole biosynthetic process from glutamate Relationships: is a type of GO:0045764; is a type of GO:0062013; is a type of GO:1901410; is a type of positive regulation of tetrapyrrole biosynthetic process [GO:1901465]; positively regulates tetrapyrrole biosynthetic process from glutamate [GO:0033526]